{
  "gene": "UniProtKB:P49619",
  "term_id": "GO:0035556",
  "gene_symbol": "DGKG",
  "gene_name": "Diacylglycerol kinase gamma",
  "term_label": "intracellular signal transduction"
}